phenolic phthiocerol biosynthetic process [GO:0097041] (biological process) Definition: The chemical reactions and pathways resulting in the formation of phenolic phthiocerol, a phthiocerol derivative having a 4-hydroxyphenyl substituent at the 29-position. Relationships: is a type of lipid biosynthetic process [GO:0008610]; is a type of GO:0046173; is a type of phenol-containing compound biosynthetic process [GO:0046189] Also known as: phenolic phthiocerol anabolism, phenolic phthiocerol biosynthesis, phenolic phthiocerol formation, phenolic phthiocerol synthesis, phenolphthiocerol biosynthesis References: PMID:9201977 Sources: GOC:dph, GOC:ecd